negative regulation of cellooligosaccharide catabolic process [GO:2000964] (biological process) Sources: GOC:mengo_curators Relationships: is_a negative regulation of catabolic process [GO:0009895]; is a type of negative regulation of carbohydrate metabolic process [GO:0045912]; is a type of regulation of cellooligosaccharide catabolic process [GO:2000963]; negatively regulates GO:2000903 Definition: Any process that stops, prevents or reduces the frequency, rate or extent of cellooligosaccharide catabolic process. Also known as: negative regulation of cellooligosaccharide catabolism